{
  "gene_name": "COMM domain-containing protein 6",
  "gene": "UniProtKB:Q7Z4G1",
  "term_label": "signal transduction",
  "term_id": "GO:0007165",
  "gene_symbol": "COMMD6"
}